{
  "term_label": "Unknown cellular component",
  "gene_symbol": "IGHV8-51-1",
  "term_id": "UNKNOWN:0003",
  "gene_name": "Probable non-functional immunoglobulin heavy variable 8-51-1",
  "gene": "UniProtKB:P0DTE2"
}